{
  "term_id": "GO:0031995",
  "gene_name": "Insulin-like growth factor-binding protein 2",
  "gene_symbol": "IGFBP2",
  "term_label": "insulin-like growth factor II binding",
  "gene": "UniProtKB:P18065"
}